{
  "gene": "UniProtKB:Q96MC4",
  "gene_symbol": "CEP295NL",
  "gene_name": "CEP295 N-terminal-like protein",
  "term_id": "GO:0005814",
  "term_label": "centriole"
}